{
  "gene": "UniProtKB:Q16620",
  "term_id": "GO:0007169",
  "gene_name": "BDNF_NT-3 growth factors receptor",
  "gene_symbol": "NTRK2",
  "term_label": "cell surface receptor protein tyrosine kinase signaling pathway"
}